{
  "term_label": "cytosol",
  "gene": "UniProtKB:P29401",
  "gene_name": "Transketolase",
  "gene_symbol": "TKT",
  "term_id": "GO:0005829"
}